{
  "term_id": "GO:0005543",
  "gene_name": "Nuclear pore glycoprotein p62",
  "gene_symbol": "NUP62",
  "gene": "UniProtKB:P37198",
  "term_label": "phospholipid binding"
}